{
  "gene": "UniProtKB:Q8WW14",
  "term_id": "UNKNOWN:0003",
  "gene_symbol": "C10orf82",
  "gene_name": "Uncharacterized protein C10orf82",
  "term_label": "Unknown cellular component"
}